alkyne biosynthetic process [GO:0043453] (biological process) Sources: GOC:jl, GOC:krc, Wikipedia:Alkyne Definition: The chemical reactions and pathways resulting in the formation of an alkyne, any acyclic branched or unbranched hydrocarbon (compound composed only of carbon and hydrogen) having a carbon-carbon triple bond and the general formula CnH2n-2. Also known as: alkyne anabolism, alkyne biosynthesis, alkyne formation, alkyne synthesis Relationships: is a type of hydrocarbon biosynthetic process [GO:0120251]